protein insertion into mitochondrial membrane [GO:0051204] (BP) Relationships: is a type of protein insertion into membrane [GO:0051205]; is a type of GO:0090151; is part of protein localization to mitochondrion [GO:0070585] Sources: GOC:ai Subtypes: protein insertion into mitochondrial inner membrane [GO:0045039], protein insertion into mitochondrial outer membrane [GO:0045040] Definition: The process that results in the incorporation of a protein into a mitochondrial membrane. Also known as: integral mitochondrial membrane protein localization, integral mitochondrial membrane protein positioning, localization of protein in mitochondrial membrane, positioning of protein in mitochondrial membrane, protein insertion into mitochondrion membrane, protein-mitochondrial membrane insertion, protein-mitochondrion membrane insertion